{
  "gene_symbol": "ORAI1",
  "gene_name": "Calcium release-activated calcium channel protein 1",
  "gene": "UniProtKB:Q96D31",
  "term_label": "membrane",
  "term_id": "GO:0016020"
}